{
  "gene_symbol": "GRAMD4",
  "gene_name": "GRAM domain-containing protein 4",
  "term_id": "UNKNOWN:0001",
  "gene": "UniProtKB:Q6IC98",
  "term_label": "Unknown molecular function"
}